{
  "gene_name": "Cadherin-3",
  "gene": "UniProtKB:P22223",
  "term_id": "GO:0005912",
  "term_label": "adherens junction",
  "gene_symbol": "CDH3"
}